adenylate cyclase binding [GO:0008179] (molecular function) Sources: GOC:jl Also known as: adenylyl cyclase binding Definition: Binding to an adenylate cyclase. Relationships: is a type of enzyme binding [GO:0019899]